{
  "term_label": "cell-cell adhesion mediated by cadherin",
  "term_id": "GO:0044331",
  "gene_symbol": "CDH3",
  "gene": "UniProtKB:P22223",
  "gene_name": "Cadherin-3"
}